{
  "term_label": "molecular carrier activity",
  "gene": "UniProtKB:Q9H3L0",
  "gene_name": "Cobalamin trafficking protein CblD",
  "term_id": "GO:0140104",
  "gene_symbol": "MMADHC"
}